hydroxylamine dehydrogenase activity [GO:0140305] (molecular function) Definition: Catalysis of the reaction: hydroxylamine + 4 Fe(III)-[cytochrome c] + H2O = 4 Fe(II)-[cytochrome c] + nitrite + 5 H+. Sources: RHEA:45032 Relationships: is a type of GO:0016662